{
  "gene_symbol": "POLR1E",
  "gene": "UniProtKB:Q9GZS1",
  "gene_name": "DNA-directed RNA polymerase I subunit RPA49",
  "term_label": "Unknown molecular function",
  "term_id": "UNKNOWN:0001"
}